{
  "gene_symbol": "RPS2",
  "gene": "UniProtKB:P15880",
  "term_id": "GO:0022627",
  "term_label": "cytosolic small ribosomal subunit",
  "gene_name": "Small ribosomal subunit protein uS5"
}